positive regulation of biosynthetic process of antibacterial peptides active against Gram-positive bacteria [GO:0006965] (biological process) References: PMID:10973475 Sources: GOC:mah Also known as: anti-Gram-positive bacterial peptide induction, anti-Gram-positive bacterial polypeptide induction, up regulation of biosynthetic process of antibacterial peptides active against Gram-positive bacteria, up-regulation of biosynthetic process of antibacterial peptides active against Gram-positive bacteria, upregulation of biosynthetic process of antibacterial peptides active against Gram-positive bacteria, activation of biosynthetic process of antibacterial peptides active against Gram-positive bacteria, stimulation of biosynthetic process of antibacterial peptides active against Gram-positive bacteria Definition: Any process that activates or increases the frequency, rate, or extent of biosynthesis of antibacterial peptides active against Gram-positive bacteria. Relationships: is_a regulation of biosynthetic process of antibacterial peptides active against Gram-positive bacteria [GO:0002816]; is a type of positive regulation of antibacterial peptide biosynthetic process [GO:0006963]; positively regulates biosynthetic process of antibacterial peptides active against Gram-positive bacteria [GO:0002815]